{
  "term_label": "Unknown molecular function",
  "gene": "UniProtKB:Q9NWQ9",
  "gene_name": "Uncharacterized protein C14orf119",
  "gene_symbol": "C14orf119",
  "term_id": "UNKNOWN:0001"
}